postsynaptic neurotransmitter receptor internalization [GO:0098884] (biological process) Sources: GOC:dos Also known as: postsynaptic neurotransmitter receptor endocytosis Regulation: regulated by regulation of postsynaptic neurotransmitter receptor internalization [GO:0099149] Relationships: is a type of regulation of postsynaptic membrane neurotransmitter receptor levels [GO:0099072]; is a type of neurotransmitter receptor internalization [GO:0099590]; is_a postsynaptic endocytosis [GO:0140239] Definition: A receptor-mediated endocytosis process that results in the internalization of a neurotransmitter receptor from the postsynaptic membrane endocytic zone into an endocytic vesicle.